{
  "term_id": "UNKNOWN:0003",
  "gene_symbol": "AVEN",
  "gene": "UniProtKB:Q9NQS1",
  "gene_name": "Cell death regulator Aven",
  "term_label": "Unknown cellular component"
}